bradykinin biosynthetic process [GO:0002936] (biological process) Definition: The chemical reactions and pathways resulting in the formation of the peptide hormone bradykinin. References: PMID:11226291 Relationships: is a type of peptide biosynthetic process [GO:0043043]; is a type of amide biosynthetic process [GO:0043604]